{
  "gene": "UniProtKB:Q9BRT9",
  "gene_symbol": "GINS4",
  "term_label": "double-strand break repair via break-induced replication",
  "term_id": "GO:0000727",
  "gene_name": "DNA replication complex GINS protein SLD5"
}